{
  "gene_symbol": "BICRAL",
  "gene_name": "BRD4-interacting chromatin-remodeling complex-associated protein-like",
  "gene": "UniProtKB:Q6AI39",
  "term_label": "positive regulation of DNA-templated transcription",
  "term_id": "GO:0045893"
}